ubiquitin protein ligase binding [GO:0031625] (molecular function) Also known as: ubiquitin ligase binding Sources: GOC:vp Relationships: is a type of ubiquitin-like protein ligase binding [GO:0044389] Definition: Binding to a ubiquitin protein ligase enzyme, any of the E3 proteins.